{
  "gene_name": "Leukocyte immunoglobulin-like receptor subfamily A member 6",
  "term_label": "cytokine-mediated signaling pathway",
  "gene_symbol": "LILRA6",
  "gene": "UniProtKB:Q6PI73",
  "term_id": "GO:0019221"
}